{
  "gene_symbol": "OGA",
  "term_label": "Unknown cellular component",
  "gene": "UniProtKB:O60502",
  "gene_name": "Protein O-GlcNAcase",
  "term_id": "UNKNOWN:0003"
}